response to cytokine [GO:0034097] (biological process) Regulation: regulated by regulation of response to cytokine stimulus [GO:0060759]; positively regulated by positive regulation of response to cytokine stimulus [GO:0060760]; negatively regulated by negative regulation of response to cytokine stimulus [GO:0060761] Also known as: response to cytokine stimulus Definition: Any process that results in a change in state or activity of a cell or an organism (in terms of movement, secretion, enzyme production, gene expression, etc.) as a result of a cytokine stimulus. Relationships: is a type of GO:1901652 Subtypes: response to type I interferon [GO:0034340], response to type II interferon [GO:0034341], GO:0034342, response to tumor necrosis factor [GO:0034612], response to interferon-alpha [GO:0035455], response to interferon-beta [GO:0035456], GO:0035962, response to macrophage colony-stimulating factor [GO:0036005], response to interleukin-3 [GO:0036015], GO:0036017, response to stem cell factor [GO:0036215], response to interleukin-1 [GO:0070555], GO:0070669, response to interleukin-4 [GO:0070670], GO:0070671, response to interleukin-15 [GO:0070672], response to interleukin-18 [GO:0070673], GO:0070741, GO:0071104, response to interleukin-11 [GO:0071105], GO:0071345, response to granulocyte macrophage colony-stimulating factor [GO:0097012], response to interleukin-32 [GO:0097395], response to interleukin-17 [GO:0097396], response to interleukin-21 [GO:0098756], response to interleukin-8 [GO:0098758], GO:0098760, GO:1990638, response to leukemia inhibitory factor [GO:1990823], GO:1990868 Sources: GOC:sl